symbiont-mediated perturbation of host translation [GO:0019057] (biological process) Sources: ISBN:0781718325 Definition: A process in which a symbiont alters or subverts translation of mRNA into protein in its host. The host is defined as the larger of the organisms involved in a symbiotic interaction. Relationships: is a type of GO:0039656 Also known as: host cell protein synthesis shutoff, regulation of host mRNA translation, regulation of host translation, modification by virus of host cell mRNA translation, modulation by virus of host translation, modulation of host translation by virus, viral perturbation of host cell mRNA translation Subtypes: symbiont-mediated suppression of host translation [GO:0039604]